{
  "gene_name": "Cilia- and flagella-associated protein 68",
  "gene": "UniProtKB:Q9H5F2",
  "term_label": "Unknown molecular function",
  "term_id": "UNKNOWN:0001",
  "gene_symbol": "CFAP68"
}